{
  "gene_name": "Probable gluconokinase",
  "gene": "UniProtKB:Q5T6J7",
  "gene_symbol": "IDNK",
  "term_id": "GO:0046316",
  "term_label": "gluconokinase activity"
}